{
  "gene": "UniProtKB:P62312",
  "gene_symbol": "LSM6",
  "gene_name": "U6 snRNA-associated Sm-like protein LSm6",
  "term_label": "maturation of SSU-rRNA",
  "term_id": "GO:0030490"
}